{
  "term_label": "vesicle docking",
  "term_id": "GO:0048278",
  "gene": "UniProtKB:O60499",
  "gene_name": "Syntaxin-10",
  "gene_symbol": "STX10"
}